organelle disassembly [GO:1903008] (biological process) Subtypes: septin ring disassembly [GO:0031107], ribosome disassembly [GO:0032790], stress granule disassembly [GO:0035617], spindle disassembly [GO:0051230], cilium disassembly [GO:0061523], kinetochore disassembly [GO:0062096], Golgi disassembly [GO:0090166], proteasome storage granule disassembly [GO:1902907], P granule disassembly [GO:1903864], chloroplast disassembly [GO:1904821], nucleus disassembly [GO:1905690], lipid droplet disassembly [GO:1905691], GO:1905692 Sources: GOC:TermGenie, GO_REF:0000079 Also known as: organelle degradation Relationships: is a type of GO:0006996; is a type of GO:0022411 Definition: The disaggregation of an organelle into its constituent components.